regulation of phosphatidylglycerol biosynthetic process [GO:1901351] (biological process) Definition: Any process that modulates the frequency, rate or extent of phosphatidylglycerol biosynthetic process. References: PMID:12869188 Sources: GOC:TermGenie, GOC:dgf Also known as: regulation of phosphatidylglycerol anabolism, regulation of phosphatidylglycerol biosynthesis, regulation of phosphatidylglycerol formation, regulation of phosphatidylglycerol synthesis Relationships: is_a regulation of phospholipid biosynthetic process [GO:0071071]; regulates phosphatidylglycerol biosynthetic process [GO:0006655] Subtypes: negative regulation of phosphatidylglycerol biosynthetic process [GO:1901352], GO:1901353